{
  "gene": "UniProtKB:Q8NGX2",
  "term_label": "plasma membrane",
  "gene_symbol": "OR2T35",
  "term_id": "GO:0005886",
  "gene_name": "Olfactory receptor 2T35"
}